negative regulation of mitochondrial translational initiation [GO:0070133] (biological process) Also known as: negative regulation of mitochondrial translation initiation Definition: Any process that stops, prevents, or reduces the frequency, rate or extent of the process preceding formation of the peptide bond between the first two amino acids of a protein in a mitochondrion. Sources: GOC:mah Relationships: is a type of negative regulation of translational initiation [GO:0045947]; is a type of regulation of mitochondrial translational initiation [GO:0070132]; negatively regulates mitochondrial translational initiation [GO:0070124]